{
  "gene_symbol": "NSUN5P2",
  "term_label": "Unknown cellular component",
  "gene_name": "Putative methyltransferase NSUN5C",
  "gene": "UniProtKB:Q63ZY6",
  "term_id": "UNKNOWN:0003"
}